nitroalkane oxidase activity [GO:0052664] (molecular function) Also known as: NAO activity, nitroalkane reductase activity, nitroalkane:oxygen oxidoreductase activity Relationships: is a type of GO:0016663 Sources: EC:1.7.3.1 Definition: Catalysis of the reaction: a primary nitroalkane + H2O + O2 = an aldehyde + H+ + H2O2 + nitrite; also converts secondary nitroalkanes to a ketone.